{
  "gene_name": "Calmodulin-regulated spectrin-associated protein 1",
  "gene": "UniProtKB:Q5T5Y3",
  "term_label": "Unknown biological process",
  "term_id": "UNKNOWN:0002",
  "gene_symbol": "CAMSAP1"
}